{
  "term_id": "GO:0050852",
  "gene_symbol": "MOG",
  "term_label": "T cell receptor signaling pathway",
  "gene_name": "Myelin-oligodendrocyte glycoprotein",
  "gene": "UniProtKB:Q16653"
}